{
  "gene_name": "Putative uncharacterized protein encoded by LINC00470",
  "term_id": "UNKNOWN:0001",
  "gene_symbol": "LINC00470",
  "term_label": "Unknown molecular function",
  "gene": "UniProtKB:Q9BZP3"
}